4-nitrophenol 2-monooxygenase activity [GO:0018601] (molecular function) Definition: Catalysis of the reaction: 4-nitrophenol + H+ + NADH + O2 = 4-nitrocatechol + H2O + NAD+. Sources: EC:1.14.13.29, RHEA:12568 Relationships: is a type of GO:0016709 Also known as: 4-nitrophenol hydroxylase activity, 4-nitrophenol,NADH:oxygen oxidoreductase (2-hydroxylating), 4-nitrophenol-2-hydroxylase activity